{
  "term_id": "GO:0031201",
  "term_label": "SNARE complex",
  "gene_symbol": "BET1L",
  "gene": "UniProtKB:Q9NYM9",
  "gene_name": "BET1-like protein"
}